{
  "term_id": "GO:0031982",
  "gene": "UniProtKB:Q7Z4J2",
  "gene_name": "Putative glycosyltransferase 6 domain-containing protein 1",
  "term_label": "vesicle",
  "gene_symbol": "GLT6D1"
}